{
  "gene": "UniProtKB:O43688",
  "gene_symbol": "PLPP2",
  "term_id": "GO:0046839",
  "gene_name": "Phospholipid phosphatase 2",
  "term_label": "phospholipid dephosphorylation"
}